{
  "term_id": "UNKNOWN:0002",
  "gene": "UniProtKB:P0DPR3",
  "gene_symbol": "TRDD1",
  "term_label": "Unknown biological process",
  "gene_name": "T cell receptor delta diversity 1"
}